{
  "gene_symbol": "FABP3",
  "term_label": "long-chain fatty acid binding",
  "term_id": "GO:0036041",
  "gene_name": "Fatty acid-binding protein, heart",
  "gene": "UniProtKB:P05413"
}